{
  "gene": "UniProtKB:Q9H5Y7",
  "gene_symbol": "SLITRK6",
  "gene_name": "SLIT and NTRK-like protein 6",
  "term_label": "positive regulation of synapse assembly",
  "term_id": "GO:0051965"
}